{
  "gene_symbol": "PTPRK",
  "gene": "UniProtKB:Q15262",
  "term_label": "signal transduction",
  "gene_name": "Receptor-type tyrosine-protein phosphatase kappa",
  "term_id": "GO:0007165"
}